growth of unicellular organism as a thread of attached cells [GO:0070783] (biological process) Regulation: regulated by regulation of growth of unicellular organism as a thread of attached cells [GO:0070784]; RO_0002212 by negative regulation of growth of unicellular organism as a thread of attached cells [GO:0070785]; positively regulated by positive regulation of growth of unicellular organism as a thread of attached cells [GO:0070786] Subtypes: pseudohyphal growth [GO:0007124], invasive filamentous growth [GO:0036267] Definition: A filamentous growth process in which cells remain attached after division and form thread-like filaments that may penetrate into a solid growth medium such as an agar plate, exhibited by unicellular fungi under certain growth conditions. Relationships: is a type of filamentous growth of a population of unicellular organisms [GO:0044182] Sources: GOC:mah, GOC:mcc